CD95 death-inducing signaling complex [GO:0031265] (cellular component) Definition: A protein complex formed upon binding of Fas/CD95/APO-1 to its ligand. The complex includes FADD/Mort1, procaspase-8/10 and c-FLIP in addition to the ligand-bound receptor. Relationships: is a type of death-inducing signaling complex [GO:0031264] Also known as: CD95 DISC, CD95 death-inducing signalling complex, Fas death-inducing signaling complex References: PMID:12628743, PMID:12655293